{
  "term_label": "cell surface receptor signaling pathway",
  "gene": "UniProtKB:A0A0K0K1D8",
  "term_id": "GO:0007166",
  "gene_name": "T cell receptor beta variable 6-1",
  "gene_symbol": "TRBV6-1"
}